{
  "term_id": "GO:0030513",
  "gene": "UniProtKB:Q96IV0",
  "gene_name": "Peptide-N(4)-(N-acetyl-beta-glucosaminyl)asparagine amidase",
  "gene_symbol": "NGLY1",
  "term_label": "positive regulation of BMP signaling pathway"
}